{
  "term_id": "GO:0004865",
  "gene": "UniProtKB:O96001",
  "gene_symbol": "PPP1R17",
  "gene_name": "Protein phosphatase 1 regulatory subunit 17",
  "term_label": "protein serine/threonine phosphatase inhibitor activity"
}